{
  "term_id": "GO:0098609",
  "gene_symbol": "CD93",
  "term_label": "cell-cell adhesion",
  "gene": "UniProtKB:Q9NPY3",
  "gene_name": "Complement component C1q receptor"
}